{
  "gene": "UniProtKB:Q13111",
  "term_label": "nucleus",
  "gene_name": "Chromatin assembly factor 1 subunit A",
  "term_id": "GO:0005634",
  "gene_symbol": "CHAF1A"
}